{
  "gene": "UniProtKB:O75061",
  "term_label": "synaptic vesicle uncoating",
  "term_id": "GO:0016191",
  "gene_name": "Putative tyrosine-protein phosphatase auxilin",
  "gene_symbol": "DNAJC6"
}